{
  "gene": "UniProtKB:Q76N89",
  "gene_symbol": "HECW1",
  "term_label": "regulation of dendrite morphogenesis",
  "gene_name": "E3 ubiquitin-protein ligase HECW1",
  "term_id": "GO:0048814"
}